negative regulation of T cell mediated immunity [GO:0002710] (biological process) Definition: Any process that stops, prevents, or reduces the frequency, rate, or extent of T cell mediated immunity. Sources: GOC:add Subtypes: negative regulation of type IV hypersensitivity [GO:0001808], negative regulation of T cell mediated cytotoxicity [GO:0001915], negative regulation of T cell antigen processing and presentation [GO:0002626], negative regulation of T cell cytokine production [GO:0002725], negative regulation of T cell mediated immune response to tumor cell [GO:0002841], negative regulation of peripheral T cell tolerance induction [GO:0002850] Also known as: down regulation of T cell mediated immunity, down-regulation of T cell mediated immunity, downregulation of T cell mediated immunity, negative regulation of T lymphocyte mediated immunity, negative regulation of T-cell mediated immunity, negative regulation of T-lymphocyte mediated immunity, inhibition of T cell mediated immunity Relationships: is a type of negative regulation of lymphocyte mediated immunity [GO:0002707]; is a type of GO:0002709; is a type of negative regulation of adaptive immune response based on somatic recombination of immune receptors built from immunoglobulin superfamily domains [GO:0002823]; negatively regulates GO:0002456